{
  "term_id": "GO:0031032",
  "term_label": "actomyosin structure organization",
  "gene": "UniProtKB:Q9NXW9",
  "gene_name": "Alpha-ketoglutarate-dependent dioxygenase alkB homolog 4",
  "gene_symbol": "ALKBH4"
}